{
  "term_id": "GO:0002250",
  "gene_symbol": "TEC",
  "term_label": "adaptive immune response",
  "gene_name": "Tyrosine-protein kinase Tec",
  "gene": "UniProtKB:P42680"
}